alpha-santalene synthase activity [GO:0102062] (molecular function) Definition: Catalysis of the reaction: 2-cis,6-cis-farnesyl diphosphate = (+)-alpha-santalene + diphosphoric acid. Relationships: is a type of carbon-oxygen lyase activity, acting on phosphates [GO:0016838] Sources: EC:4.2.3.50, GOC:pz